{
  "gene": "UniProtKB:Q8NFJ9",
  "term_id": "GO:0005813",
  "term_label": "centrosome",
  "gene_name": "Bardet-Biedl syndrome 1 protein",
  "gene_symbol": "BBS1"
}